ecdysis-triggering hormone activity [GO:0008255] (molecular function) Definition: The action characteristic of ecdysis-triggering hormone, a peptide hormone that, upon receptor binding, initiates pre-ecdysis and ecdysis (i.e. cuticle shedding) through direct action on the central nervous system. References: PMID:9020043 Sources: GOC:mah Relationships: is a type of neuropeptide hormone activity [GO:0005184]